{
  "term_id": "GO:0090160",
  "gene_name": "AP-4 complex subunit mu-1",
  "gene_symbol": "AP4M1",
  "gene": "UniProtKB:O00189",
  "term_label": "Golgi to lysosome transport"
}